{
  "term_label": "cell surface receptor signaling pathway",
  "gene_symbol": "TRBV6-7",
  "gene_name": "Probable non-functional T cell receptor beta variable 6-7",
  "term_id": "GO:0007166",
  "gene": "UniProtKB:A0A0A0MS04"
}